membrane organization [GO:0061024] (biological process) Subtypes: postsynaptic membrane organization [GO:0001941], GO:0006900, nuclear envelope organization [GO:0006998], GO:0007006, plasma membrane organization [GO:0007009], membrane addition at site of cytokinesis [GO:0007107], plastid membrane organization [GO:0009668], membrane invagination [GO:0010324], membrane disassembly [GO:0030397], GO:0031579, GO:0032594, GO:0033292, GO:0045161, Golgi vesicle bud deformation and release [GO:0048198], synaptic vesicle membrane organization [GO:0048499], membrane fusion [GO:0061025], GO:0061952, spore membrane bending pathway [GO:0070583], membrane assembly [GO:0071709], nuclear membrane organization [GO:0071763], GO:0090148, endoplasmic reticulum membrane organization [GO:0090158], regulation of membrane lipid distribution [GO:0097035], GO:0097090, lysosomal membrane organization [GO:0097212], membrane tubulation [GO:0097749], GO:0097753, trans-Golgi network membrane organization [GO:0098629], mitotic nuclear membrane biogenesis [GO:0101026], intermembrane lipid transfer [GO:0120009] Definition: A process which results in the assembly, arrangement of constituent parts, or disassembly of a membrane. A membrane is a double layer of lipid molecules that encloses all cells, and, in eukaryotes, many organelles; may be a single or double lipid bilayer; also includes associated proteins. Relationships: is a type of cellular component organization [GO:0016043] Also known as: cellular membrane organisation, cellular membrane organization, membrane organisation, membrane organization and biogenesis, single-organism membrane organization Sources: GOC:dph, GOC:tb